{
  "term_label": "RNA polymerase II cis-regulatory region sequence-specific DNA binding",
  "gene_symbol": "GSC2",
  "term_id": "GO:0000978",
  "gene_name": "Homeobox protein goosecoid-2",
  "gene": "UniProtKB:O15499"
}